{
  "term_label": "DNA helicase activity",
  "gene_name": "Putative ATP-dependent RNA helicase DDX12",
  "term_id": "GO:0003678",
  "gene": "UniProtKB:Q92771",
  "gene_symbol": "DDX12P"
}